{
  "term_label": "proteasome-mediated ubiquitin-dependent protein catabolic process",
  "term_id": "GO:0043161",
  "gene": "UniProtKB:O94889",
  "gene_symbol": "KLHL18",
  "gene_name": "Kelch-like protein 18"
}